{
  "term_id": "GO:0001580",
  "gene_symbol": "RTP4",
  "term_label": "detection of chemical stimulus involved in sensory perception of bitter taste",
  "gene_name": "Receptor-transporting protein 4",
  "gene": "UniProtKB:Q96DX8"
}